transcription termination site sequence-specific DNA binding [GO:0001147] (molecular function) Relationships: is a type of GO:0000976; BFO_0000050 DNA-templated transcription termination [GO:0006353] Also known as: bacterial-type RNA polymerase termination site sequence-specific DNA binding, mitochondrial RNA polymerase termination site sequence-specific DNA binding, mitochondrial RNA polymerase terminator site sequence-specific DNA binding transcription factor activity, transcription factor activity, mitochondrial RNA polymerase terminator site sequence-specific binding, transcription termination site DNA binding Note: Transcription termination sites can be recognized by the RNA polymerase (RNAP) itself or by another protein which interacts with the RNAP to promote transcription termination. Note that not all genes have a DNA specific sequence that functions as a termination site; for most mRNAs transcribed by RNAP II termination is not mediated by a specific termination sequence, but is coupled to polyadenylation. Definition: Binding to a sequence of DNA that promotes termination by RNA polymerase. The transcribed region might be described as a gene, cistron, or operon. References: PMID:18280161, PMID:18391175 Sources: GOC:txnOH